5-phosphoribosyl 1-pyrophosphate pyrophosphatase activity [GO:0043135] (molecular function) Relationships: is a type of pyrophosphatase activity [GO:0016462] Also known as: PRPP pyrophosphatase activity Definition: Catalysis of the reaction: 5-phospho-alpha-D-ribose 1-diphosphate + H2O = ribose 1,5 bisphosphate + phosphate + H+. References: PMID:12370170 Sources: MetaCyc:RXN-10969